response to abscisic acid [GO:0009737] (biological process) Relationships: is a type of response to hormone [GO:0009725]; is a type of response to lipid [GO:0033993]; is a type of response to alcohol [GO:0097305] Sources: GOC:jl Subtypes: detection of abscisic acid stimulus [GO:0009724], cellular response to abscisic acid stimulus [GO:0071215] Definition: Any process that results in a change in state or activity of a cell or an organism (in terms of movement, secretion, enzyme production, gene expression, etc.) as a result of an abscisic acid stimulus. Also known as: response to abscisic acid stimulus